purine-rich negative regulatory element binding [GO:0032422] (molecular function) Definition: Binding to a 30-bp purine-rich negative regulatory element; the best characterized such element is found in the first intronic region of the rat cardiac alpha-myosin heavy chain gene, and contains two palindromic high-affinity Ets-binding sites (CTTCCCTGGAAG). The presence of this element restricts expression of the gene containing it to cardiac myocytes. References: PMID:9819411 Sources: GOC:mah Also known as: PNR element binding Relationships: is a type of transcription cis-regulatory region binding [GO:0000976]